host cell filopodium [GO:0044176] (cellular component) Sources: GOC:jl Definition: Thin, stiff protrusion extended by the leading edge of a motile host cell such as a crawling fibroblast or amoeba, or an axonal growth cone; usually approximately 0.1 um wide, 5-10 um long, can be up to 50 um long in axon growth cones; contains a loose bundle of about 20 actin filaments oriented with their plus ends pointing outward. Relationships: is a type of GO:0044157 Also known as: host filopodium